{
  "term_label": "DNA-binding transcription factor activity, RNA polymerase II-specific",
  "gene_symbol": "PROP1",
  "gene_name": "Homeobox protein prophet of Pit-1",
  "gene": "UniProtKB:O75360",
  "term_id": "GO:0000981"
}